{
  "gene_name": "Fibroblast growth factor 10",
  "term_label": "positive regulation of MAPK cascade",
  "gene_symbol": "FGF10",
  "gene": "UniProtKB:O15520",
  "term_id": "GO:0043410"
}